axonemal A tubule inner sheath [GO:0160111] (cellular component) References: PMID:29430673, PMID:37295417 Sources: GOC:krc Definition: A structural network of microtubule inner proteins (MIPs) located inside the lumen of the A tubule of the axonemal microtubule doublet that helps stabilize the A tubule. Relationships: is a type of cellular anatomical structure [GO:0110165]; is part of A axonemal microtubule [GO:0097649]; is part of axonemal microtubule doublet inner sheath [GO:0160110]